interleukin-23 binding [GO:0042019] (molecular function) Relationships: is a type of cytokine binding [GO:0019955] Also known as: IL-23 binding Sources: GOC:jl Definition: Binding to interleukin-23.